{
  "gene": "UniProtKB:Q9UMZ2",
  "gene_symbol": "SYNRG",
  "term_id": "UNKNOWN:0001",
  "gene_name": "Synergin gamma",
  "term_label": "Unknown molecular function"
}